arginine deiminase activity [GO:0016990] (molecular function) Also known as: L-arginine deiminase activity, L-arginine iminohydrolase activity, arginine dihydrolase activity, citrulline iminase activity Definition: Catalysis of the reaction: L-arginine + H2O = L-citrulline + NH3. Sources: EC:3.5.3.6 Relationships: is a type of hydrolase activity, acting on carbon-nitrogen (but not peptide) bonds, in linear amidines [GO:0016813]